{
  "gene_name": "Olfactory receptor 11H6",
  "gene_symbol": "OR11H6",
  "term_label": "Unknown molecular function",
  "term_id": "UNKNOWN:0001",
  "gene": "UniProtKB:Q8NGC7"
}